{
  "term_id": "GO:0007052",
  "gene_symbol": "WDR62",
  "term_label": "mitotic spindle organization",
  "gene_name": "WD repeat-containing protein 62",
  "gene": "UniProtKB:O43379"
}